{
  "gene_name": "Leucine-rich PPR motif-containing protein, mitochondrial",
  "term_label": "nucleus",
  "term_id": "GO:0005634",
  "gene": "UniProtKB:P42704",
  "gene_symbol": "LRPPRC"
}